{
  "gene_symbol": "TLR7",
  "gene": "UniProtKB:Q9NYK1",
  "gene_name": "Toll-like receptor 7",
  "term_id": "GO:0034154",
  "term_label": "toll-like receptor 7 signaling pathway"
}